{
  "gene_symbol": "TRBV5-5",
  "term_id": "GO:0005886",
  "gene_name": "T cell receptor beta variable 5-5",
  "gene": "UniProtKB:A0A597",
  "term_label": "plasma membrane"
}